{
  "term_id": "UNKNOWN:0003",
  "gene": "UniProtKB:Q9UEW3",
  "gene_symbol": "MARCO",
  "term_label": "Unknown cellular component",
  "gene_name": "Macrophage receptor MARCO"
}